{
  "term_label": "regulation of transcription by RNA polymerase II",
  "term_id": "GO:0006357",
  "gene_symbol": "ZNF436",
  "gene_name": "Zinc finger protein 436",
  "gene": "UniProtKB:Q9C0F3"
}